{
  "term_label": "receptor complex",
  "gene": "UniProtKB:P78552",
  "gene_name": "Interleukin-13 receptor subunit alpha-1",
  "term_id": "GO:0043235",
  "gene_symbol": "IL13RA1"
}